{
  "gene": "UniProtKB:Q8NGR9",
  "gene_name": "Olfactory receptor 1N2",
  "gene_symbol": "OR1N2",
  "term_label": "olfactory receptor activity",
  "term_id": "GO:0004984"
}